{
  "term_id": "GO:0004842",
  "gene_name": "Peroxisome assembly protein 12",
  "gene_symbol": "PEX12",
  "gene": "UniProtKB:O00623",
  "term_label": "ubiquitin-protein transferase activity"
}